{
  "gene_symbol": "TRPM4",
  "term_label": "metal ion transport",
  "term_id": "GO:0030001",
  "gene": "UniProtKB:Q8TD43",
  "gene_name": "Transient receptor potential cation channel subfamily M member 4"
}